{
  "gene": "UniProtKB:Q16280",
  "gene_symbol": "CNGA2",
  "gene_name": "Cyclic nucleotide-gated olfactory channel",
  "term_label": "intracellularly cAMP-activated cation channel activity",
  "term_id": "GO:0005222"
}